isoprenoid diphosphate phosphatase activity [GO:0106405] (molecular function) Definition: Catalysis of the dephosphorylation of isoprenoid diphosphates. Relationships: is a type of pyrophosphatase activity [GO:0016462] Subtypes: polyprenyl diphosphate phosphatase activity [GO:0120556] References: PMID:33246356